{
  "gene": "UniProtKB:Q6UDR6",
  "term_id": "UNKNOWN:0002",
  "gene_symbol": "SPINT4",
  "gene_name": "Kunitz-type protease inhibitor 4",
  "term_label": "Unknown biological process"
}